{
  "term_id": "GO:0005634",
  "term_label": "nucleus",
  "gene_name": "Insulin gene enhancer protein ISL-2",
  "gene_symbol": "ISL2",
  "gene": "UniProtKB:Q96A47"
}